{
  "term_id": "GO:1990112",
  "gene": "UniProtKB:Q9BQ70",
  "term_label": "RQC complex",
  "gene_symbol": "TCF25",
  "gene_name": "Ribosome quality control complex subunit TCF25"
}